NADPH-hemoprotein reductase activity [GO:0003958] (MF) Definition: Catalysis of the reaction: NADPH + H+ + n oxidized hemoprotein = NADP+ + n reduced hemoprotein. Sources: EC:1.6.2.4 Also known as: NADPH-ferrihemoprotein reductase activity, NADPH:cytochrome P450 reductase activity, NADPH:cytochrome c reductase activity, NADP--cytochrome c reductase activity, NADP--cytochrome reductase activity, NADPH--cytochrome P450 oxidoreductase activity, NADPH--cytochrome P450 reductase activity, NADPH--cytochrome c oxidoreductase activity, NADPH--cytochrome c reductase activity, NADPH--ferricytochrome c oxidoreductase activity, NADPH--ferrihemoprotein reductase activity, NADPH-dependent cytochrome c reductase activity, NADPH:P450 reductase activity, TPNH(2) cytochrome c reductase activity, TPNH-cytochrome c reductase activity, cytochrome P450 reductase activity, cytochrome c reductase (reduced nicotinamide adenine dinucleotide phosphate, NADPH, NADPH-dependent) activity, dihydroxynicotinamide adenine dinucleotide phosphate-cytochrome c reductase activity, reduced nicotinamide adenine dinucleotide phosphate-cytochrome c reductase activity, reductase, cytochrome c (reduced nicotinamide adenine dinucleotide phosphate) activity, CPR activity, FAD-cytochrome c reductase activity, NADPH-cytochrome P-450 oxidoreductase activity, NADPH-cytochrome p-450 reductase activity, NADPH:P-450 reductase activity, NADPH:ferrihemoprotein oxidoreductase activity, NADPH:hemoprotein oxidoreductase activity, POR, TPNH2 cytochrome c reductase activity, aldehyde reductase (NADPH-dependent) activity, cytochrome P-450 reductase activity, ferrihemoprotein P-450 reductase activity Relationships: is a type of oxidoreductase activity, acting on NAD(P)H, heme protein as acceptor [GO:0016653]